{
  "gene_symbol": "GRIK3",
  "gene": "UniProtKB:Q13003",
  "term_id": "GO:1904315",
  "term_label": "transmitter-gated monoatomic ion channel activity involved in regulation of postsynaptic membrane potential",
  "gene_name": "Glutamate receptor ionotropic, kainate 3"
}